{
  "gene_name": "Stonin-2",
  "gene": "UniProtKB:Q8WXE9",
  "term_id": "GO:0072583",
  "term_label": "clathrin-dependent endocytosis",
  "gene_symbol": "STON2"
}